{
  "term_id": "GO:0004386",
  "term_label": "helicase activity",
  "gene": "UniProtKB:Q7Z478",
  "gene_name": "ATP-dependent RNA helicase DHX29",
  "gene_symbol": "DHX29"
}